autophagosome-endosome fusion [GO:0061910] (biological process) Relationships: is_a vesicle fusion [GO:0006906]; is part of macroautophagy [GO:0016236] References: PMID:24219988 Definition: The process in which an autophagosome fuses with an endosome to create an intermediate autophagic organelle called amphisome.